regulation of vascular permeability involved in acute inflammatory response [GO:0002528] (BP) Definition: Any process that modulates the extent to which blood vessels can be pervaded by fluid contributing to an acute inflammatory response. Sources: GOC:jal Also known as: regulation of vascular permeability during acute inflammatory response Relationships: is a type of regulation of vascular permeability [GO:0043114]; is part of acute inflammatory response [GO:0002526]